{
  "gene_name": "Core histone macro-H2A.1",
  "gene": "UniProtKB:O75367",
  "term_id": "GO:0031507",
  "gene_symbol": "MACROH2A1",
  "term_label": "heterochromatin formation"
}